{
  "term_id": "UNKNOWN:0002",
  "gene_symbol": "PHGR1",
  "gene_name": "Proline, histidine and glycine-rich protein 1",
  "gene": "UniProtKB:C9JFL3",
  "term_label": "Unknown biological process"
}